{
  "gene": "UniProtKB:P56706",
  "term_label": "cell fate commitment",
  "gene_symbol": "WNT7B",
  "term_id": "GO:0045165",
  "gene_name": "Protein Wnt-7b"
}